{
  "gene_symbol": "NEDD4",
  "term_id": "GO:0019871",
  "term_label": "sodium channel inhibitor activity",
  "gene_name": "E3 ubiquitin-protein ligase NEDD4",
  "gene": "UniProtKB:P46934"
}